{
  "gene_symbol": "SNAP91",
  "term_label": "clathrin heavy chain binding",
  "term_id": "GO:0032050",
  "gene": "UniProtKB:O60641",
  "gene_name": "Clathrin coat assembly protein AP180"
}